{
  "gene_symbol": "FHOD3",
  "term_label": "sarcomere organization",
  "term_id": "GO:0045214",
  "gene": "UniProtKB:Q2V2M9",
  "gene_name": "FH1_FH2 domain-containing protein 3"
}